negative regulation of protein acetylation [GO:1901984] (biological process) Also known as: down regulation of protein acetylation, down regulation of protein amino acid acetylation, down-regulation of protein acetylation, down-regulation of protein amino acid acetylation, downregulation of protein acetylation, downregulation of protein amino acid acetylation, negative regulation of protein amino acid acetylation, inhibition of protein acetylation, inhibition of protein amino acid acetylation Subtypes: GO:1904664, negative regulation of peptidyl-lysine acetylation [GO:2000757] Definition: Any process that stops, prevents or reduces the frequency, rate or extent of protein acetylation. Relationships: is a type of negative regulation of protein modification process [GO:0031400]; is a type of regulation of protein acetylation [GO:1901983]; negatively regulates protein acetylation [GO:0006473] References: PMID:22117195 Sources: GOC:TermGenie